{
  "gene_name": "POU domain, class 4, transcription factor 1",
  "term_id": "UNKNOWN:0003",
  "term_label": "Unknown cellular component",
  "gene": "UniProtKB:Q01851",
  "gene_symbol": "POU4F1"
}